endoplasmic reticulum tubular network organization [GO:0071786] (BP) Regulation: regulated by GO:1903371; negatively regulated by negative regulation of endoplasmic reticulum tubular network organization [GO:1903372]; positively regulated by positive regulation of endoplasmic reticulum tubular network organization [GO:1903373] Relationships: is a type of GO:0007029 Also known as: ER tubular network organisation, ER tubular network organization, endoplasmic reticulum tubular network organisation Subtypes: endoplasmic reticulum tubular network formation [GO:0071787], endoplasmic reticulum tubular network maintenance [GO:0071788], endoplasmic reticulum tubular network membrane organization [GO:1990809] References: PMID:16469703, PMID:20434336 Sources: GOC:vw Definition: A process that is carried out at the cellular level which results in the assembly, arrangement of constituent parts, or disassembly of the endoplasmic reticulum (ER) tubular network. The ER tubular network is the ER part that that has membranes with high curvature in cross-section.